{
  "gene_name": "2'-5'-oligoadenylate synthase 1",
  "gene_symbol": "OAS1",
  "term_label": "membrane",
  "gene": "UniProtKB:P00973",
  "term_id": "GO:0016020"
}